{
  "term_label": "Unknown biological process",
  "term_id": "UNKNOWN:0002",
  "gene_symbol": "LRCOL1",
  "gene_name": "Leucine-rich colipase-like protein 1",
  "gene": "UniProtKB:A6NCL2"
}